endocrocin biosynthetic process [GO:1900602] (biological process) Also known as: endocrocin anabolism, endocrocin biosynthesis, endocrocin formation, endocrocin synthesis Definition: The chemical reactions and pathways resulting in the formation of endocrocin. Regulation: regulated by regulation of endocrocin biosynthetic process [GO:1900667]; negatively regulated by negative regulation of endocrocin biosynthetic process [GO:1900668]; positively regulated by GO:1900669 Sources: GOC:TermGenie, GOC:di Relationships: is a type of ketone biosynthetic process [GO:0042181]; is a type of secondary metabolite biosynthetic process [GO:0044550]; is a type of phenol-containing compound biosynthetic process [GO:0046189]; is a type of carboxylic acid biosynthetic process [GO:0046394]